choline biosynthetic process via CDP-choline [GO:0033323] (biological process) Relationships: is a type of choline biosynthetic process [GO:0042425] Definition: The chemical reactions and pathways resulting in the formation of choline (2-hydroxyethyltrimethylammonium), via the intermediate CDP-choline. Also known as: choline anabolism via CDP-choline, choline biosynthesis via CDP-choline, choline formation via CDP-choline, choline synthesis via CDP-choline Sources: GOC:mah, MetaCyc:PWY-3561